{
  "gene_symbol": "CAP1",
  "term_id": "GO:0007015",
  "gene": "UniProtKB:Q01518",
  "term_label": "actin filament organization",
  "gene_name": "Adenylyl cyclase-associated protein 1"
}